{
  "gene_name": "Histone lysine demethylase PHF8",
  "gene": "UniProtKB:Q9UPP1",
  "term_id": "GO:0032452",
  "term_label": "histone demethylase activity",
  "gene_symbol": "PHF8"
}